{
  "term_label": "basolateral plasma membrane",
  "gene_name": "Solute carrier organic anion transporter family member 1B3",
  "gene_symbol": "SLCO1B3",
  "gene": "UniProtKB:Q9NPD5",
  "term_id": "GO:0016323"
}